poly(alpha-L-guluronate) lyase activity [GO:0047491] (molecular function) Relationships: is a type of carbon-oxygen lyase activity, acting on polysaccharides [GO:0016837] Sources: EC:4.2.2.11 Definition: Catalysis of the reaction: polysaccharides containing a terminal alpha-L-guluronate group = oligosaccharides with 4-deoxy-alpha-L-erythro-hex-4-enuronosyl end. This reaction is the eliminative cleavage of polysaccharides containing a terminal a-L-guluronate group, to give oligopolysaccharides with 4-deoxy-a-L-erythro-hex-4-enuronosyl groups at their nonreducing ends. Also known as: L-guluronan lyase activity, L-guluronate lyase activity, alginase II activity, guluronate lyase activity, poly(alpha-L-1,4-guluronide) exo-lyase activity, poly-alpha-L-guluronate lyase activity, polyguluronate-specific alginate lyase activity